{
  "gene": "UniProtKB:Q86V25",
  "term_id": "UNKNOWN:0001",
  "gene_name": "Tubulinyl-Tyr carboxypeptidase 2",
  "term_label": "Unknown molecular function",
  "gene_symbol": "VASH2"
}